{
  "term_id": "UNKNOWN:0003",
  "term_label": "Unknown cellular component",
  "gene_name": "Xaa-Pro dipeptidase",
  "gene": "UniProtKB:P12955",
  "gene_symbol": "PEPD"
}